{
  "term_id": "GO:0000209",
  "term_label": "protein polyubiquitination",
  "gene": "UniProtKB:Q14669",
  "gene_name": "E3 ubiquitin-protein ligase TRIP12",
  "gene_symbol": "TRIP12"
}